{
  "term_label": "Unknown molecular function",
  "gene": "UniProtKB:P01593",
  "gene_name": "Immunoglobulin kappa variable 1D-33",
  "term_id": "UNKNOWN:0001",
  "gene_symbol": "IGKV1D-33"
}